alphaPDGFR-PLC-gamma-1-PI3K-SHP-2 complex [GO:0070719] (cellular component) Also known as: PDGFRA-PLC-gamma-1-PI3K-SHP-2 complex, PDGF stimulated References: PMID:8943348 Sources: GOC:mah Relationships: is a type of GO:0098797 Definition: A protein complex that contains the platelet-derived growth factor alpha receptor (alphaPDGFR; PDGFRA), phospholipase C-gamma-1 (PLC-gamma-1), phosphatidylinositol 3-kinase (PI3K) and the adaptor protein SHP-2, and is involved signaling via the PDGFR signaling pathway.